regulation of monoatomic anion transport [GO:0044070] (biological process) Definition: Any process that modulates the frequency, rate or extent of the directed movement of anions, atoms or small molecules with a net negative charge into, out of or within a cell, or between cells, by means of some agent such as a transporter or pore. Sources: GOC:jl Subtypes: negative regulation of monoatomic anion transport [GO:1903792], GO:1903793, GO:1903959, regulation of iodide transport [GO:1904201], regulation of chloride transport [GO:2001225] Also known as: regulation of anion transport Relationships: is a type of regulation of monoatomic ion transport [GO:0043269]; regulates monoatomic anion transport [GO:0006820]